{
  "gene_symbol": "PLA2G2F",
  "term_id": "GO:0042130",
  "gene_name": "Group IIF secretory phospholipase A2",
  "term_label": "negative regulation of T cell proliferation",
  "gene": "UniProtKB:Q9BZM2"
}